{
  "gene_symbol": "CFAP74",
  "term_id": "UNKNOWN:0003",
  "term_label": "Unknown cellular component",
  "gene_name": "Cilia- and flagella-associated protein 74",
  "gene": "UniProtKB:Q9C0B2"
}